{
  "gene": "UniProtKB:Q9BX66",
  "term_id": "GO:0031589",
  "gene_name": "Sorbin and SH3 domain-containing protein 1",
  "gene_symbol": "SORBS1",
  "term_label": "cell-substrate adhesion"
}